{
  "gene_symbol": "PAX7",
  "term_label": "DNA-binding transcription factor activity, RNA polymerase II-specific",
  "term_id": "GO:0000981",
  "gene_name": "Paired box protein Pax-7",
  "gene": "UniProtKB:P23759"
}